cephalosporin C metabolic process [GO:1901266] (BP) Also known as: cephalosporin C metabolism Sources: GOC:TermGenie, GOC:yaf, UniPathway:UPA00172 Subtypes: cephalosporin C catabolic process [GO:1901267], cephalosporin C biosynthetic process [GO:1901268] Relationships: is a type of sulfur compound metabolic process [GO:0006790]; is a type of GO:0019752; is a type of lactam metabolic process [GO:0072338] Definition: The chemical reactions and pathways involving cephalosporin C.